{
  "gene": "UniProtKB:Q86V71",
  "gene_symbol": "ZNF429",
  "term_id": "GO:0000981",
  "term_label": "DNA-binding transcription factor activity, RNA polymerase II-specific",
  "gene_name": "Zinc finger protein 429"
}